{
  "term_label": "spermidine deacetylation",
  "gene_name": "Polyamine deacetylase HDAC10",
  "term_id": "GO:0106048",
  "gene_symbol": "HDAC10",
  "gene": "UniProtKB:Q969S8"
}